6-phosphofructo-2-kinase/fructose-2,6-biphosphatase complex [GO:0043540] (cellular component) Also known as: 6-phosphofructo-2-kinase/fructose-2,6-biphosphatase 1 complex, 6-phosphofructo-2-kinase/fructose-2,6-biphosphatase 2 complex, 6-phosphofructo-2-kinase/fructose-2,6-biphosphatase 3 complex, 6-phosphofructo-2-kinase/fructose-2,6-biphosphatase 4 complex Relationships: is a type of transferase complex, transferring phosphorus-containing groups [GO:0061695]; is part of GO:0005829 Definition: A homodimeric, bifunctional enzyme complex which catalyzes the synthesis and degradation of fructose 2,6-bisphosphate, and is required for both glycolysis and gluconeogenesis. Note: Note that we use this single class to represent all 4 isoforms of this complex. We decided to do this because the isoforms do not differ in function, rather in expression and regulation. We may want to revisit this in future. Sources: GOC:jl, GOC:so